positive regulation of toll-like receptor 13 signaling pathway [GO:0034181] (biological process) Also known as: positive regulation of TLR13 signaling pathway, positive regulation of toll-like receptor 13 signalling pathway References: PMID:16551253, PMID:17328678 Sources: GOC:add Definition: Any process that activates or increases the frequency, rate, or extent of toll-like receptor 13 signaling pathway. Relationships: is a type of regulation of toll-like receptor 13 signaling pathway [GO:0034179]; is a type of positive regulation of pattern recognition receptor signaling pathway [GO:0062208]; is a type of positive regulation of intracellular signal transduction [GO:1902533]; RO_0002213 toll-like receptor 13 signaling pathway [GO:0034178]